{
  "gene": "UniProtKB:Q9Y3M2",
  "term_label": "Unknown molecular function",
  "term_id": "UNKNOWN:0001",
  "gene_symbol": "CBY1",
  "gene_name": "Protein chibby homolog 1"
}